{
  "gene": "UniProtKB:P01589",
  "gene_name": "Interleukin-2 receptor subunit alpha",
  "term_id": "GO:0019976",
  "gene_symbol": "IL2RA",
  "term_label": "interleukin-2 binding"
}